{
  "term_label": "nucleus",
  "gene_symbol": "ZNF584",
  "gene_name": "Zinc finger protein 584",
  "gene": "UniProtKB:Q8IVC4",
  "term_id": "GO:0005634"
}